{
  "gene": "UniProtKB:Q8N7P3",
  "gene_symbol": "CLDN22",
  "term_id": "GO:0005886",
  "term_label": "plasma membrane",
  "gene_name": "Claudin-22"
}